{
  "term_label": "positive regulation of apoptotic process",
  "gene_symbol": "AIFM2",
  "gene": "UniProtKB:Q9BRQ8",
  "gene_name": "Ferroptosis suppressor protein 1",
  "term_id": "GO:0043065"
}